{
  "term_id": "UNKNOWN:0003",
  "gene": "UniProtKB:A2RRL7",
  "gene_name": "Transmembrane protein 213",
  "term_label": "Unknown cellular component",
  "gene_symbol": "TMEM213"
}